{
  "term_label": "cell migration",
  "gene_name": "Tyrosine-protein kinase Mer",
  "gene_symbol": "MERTK",
  "term_id": "GO:0016477",
  "gene": "UniProtKB:Q12866"
}